{
  "term_id": "GO:0003729",
  "gene_name": "Serine_arginine-rich splicing factor 2",
  "gene_symbol": "SRSF2",
  "gene": "UniProtKB:Q01130",
  "term_label": "mRNA binding"
}